{
  "gene_name": "Cationic amino acid transporter 3",
  "term_id": "GO:0006865",
  "gene_symbol": "SLC7A3",
  "term_label": "amino acid transport",
  "gene": "UniProtKB:Q8WY07"
}